{
  "term_label": "humoral immune response",
  "gene": "UniProtKB:P01563",
  "gene_symbol": "IFNA2",
  "gene_name": "Interferon alpha-2",
  "term_id": "GO:0006959"
}